pronephros morphogenesis [GO:0072114] (BP) Sources: GOC:mtg_kidney_jan10 Relationships: is a type of kidney morphogenesis [GO:0060993]; is part of pronephros development [GO:0048793] Subtypes: head kidney morphogenesis [GO:0072115] Definition: The process in which the anatomical structures of the pronephros are generated and organized. In mammals, the pronephros is the first of the three embryonic kidneys to be established and exists only transiently. In lower vertebrates such as fish and amphibia, the pronephros is the fully functional embryonic kidney and is indispensable for larval life. Also known as: pronephric kidney morphogenesis